viral translational termination-reinitiation [GO:0075525] (BP) Note: This term is intended to annotate gene products involved in the process of viral translational termination-reinitiation, not viral proteins produced by this translation process. References: PMID:18631147, PMID:18824510 Sources: GOC:bf, GOC:ch, GOC:jl, VZ:858 Relationships: is a type of viral process [GO:0016032]; is part of viral translation [GO:0019081] Also known as: termination reinitiation involved in viral translation, viral translation involving termination re-initiation, viral translation involving termination-reinitiation, viral translation involving translational stop-start Definition: A process which occurs as part of viral mRNA translation which allows expression of a downstream open reading frame (ORF) in a dicistronic mRNA. In this process, ribosomes translate the upstream ORF but following termination, a proportion of 40S subunits remain tethered to the mRNA and go on to re-initiate translation at the start codon of the downstream ORF.